{
  "gene": "UniProtKB:Q8IXU6",
  "term_label": "Unknown cellular component",
  "gene_symbol": "SLC35F2",
  "term_id": "UNKNOWN:0003",
  "gene_name": "Solute carrier family 35 member F2"
}